gerontoplast [GO:0034400] (cellular component) Definition: A plastid found in senescing, formerly green tissues that is derived from a chloroplast that undergoes an organized developmental program of senescence. Relationships: is_a plastid [GO:0009536] References: PMID:12654863, PMID:24668747